{
  "term_id": "GO:0030896",
  "term_label": "checkpoint clamp complex",
  "gene_symbol": "RAD9B",
  "gene": "UniProtKB:Q6WBX8",
  "gene_name": "Cell cycle checkpoint control protein RAD9B"
}